regulation of hepatocyte proliferation [GO:2000345] (biological process) Subtypes: negative regulation of hepatocyte proliferation [GO:2000346], positive regulation of hepatocyte proliferation [GO:2000347] Sources: GOC:BHF, GOC:mah Definition: Any process that modulates the frequency, rate or extent of hepatocyte proliferation. Relationships: is a type of GO:0050678; regulates GO:0072574